{
  "gene_symbol": "ROM1",
  "gene_name": "Rod outer segment membrane protein 1",
  "term_id": "GO:0005886",
  "gene": "UniProtKB:Q03395",
  "term_label": "plasma membrane"
}